{
  "term_id": "UNKNOWN:0001",
  "term_label": "Unknown molecular function",
  "gene_symbol": "C5orf60",
  "gene_name": "Uncharacterized protein C5orf60",
  "gene": "UniProtKB:A6NFR6"
}